phenylalanine ammonia-lyase activity [GO:0045548] (molecular function) Sources: RHEA:21384 Relationships: is a type of ammonia-lyase activity [GO:0016841] Definition: Catalysis of the reaction: L-phenylalanine = NH4 + trans-cinnamate. Also known as: PAL activity, L-phenylalanine ammonia-lyase activity, phe ammonia-lyase activity, phenylalanine ammonium-lyase activity, phenylalanine deaminase activity